{
  "gene_name": "Isocitrate dehydrogenase [NAD] subunit gamma, mitochondrial",
  "gene": "UniProtKB:P51553",
  "term_label": "isocitrate metabolic process",
  "term_id": "GO:0006102",
  "gene_symbol": "IDH3G"
}